N-terminal peptidyl-alanine trimethylation [GO:0018012] (biological process) Sources: RESID:AA0062 Relationships: is a type of GO:0018011 Definition: The trimethylation of the N-terminal alanine of proteins to form the derivative peptidyl-N,N,N-trimethyl-L-alanine.